{
  "term_id": "UNKNOWN:0002",
  "gene": "UniProtKB:O15194",
  "term_label": "Unknown biological process",
  "gene_name": "CTD small phosphatase-like protein",
  "gene_symbol": "CTDSPL"
}